response to glial cell derived neurotrophic factor [GO:1990790] (biological process) References: PMID:20877310 Also known as: response to ATF, response to GDNF, response to astrocyte-derived trophic factor Definition: Any process that results in a change in state or activity of a cell or an organism (in terms of movement, secretion, enzyme production, gene expression, etc.) as a result of a glial cell derived neurotrophic factor stimulus. Relationships: is a type of response to growth factor [GO:0070848] Subtypes: cellular response to glial cell derived neurotrophic factor [GO:1990792]